{
  "term_label": "transcription elongation factor complex",
  "term_id": "GO:0008023",
  "gene_name": "Transcription elongation factor SPT6",
  "gene": "UniProtKB:Q7KZ85",
  "gene_symbol": "SUPT6H"
}